{
  "gene_name": "Myomesin-2",
  "term_label": "M band",
  "gene": "UniProtKB:P54296",
  "gene_symbol": "MYOM2",
  "term_id": "GO:0031430"
}